{
  "term_id": "GO:0015808",
  "gene_symbol": "SLC36A4",
  "gene_name": "Neutral amino acid uniporter 4",
  "term_label": "L-alanine transport",
  "gene": "UniProtKB:Q6YBV0"
}